{
  "gene_name": "Hyaluronidase PH-20",
  "term_id": "GO:0030214",
  "gene_symbol": "SPAM1",
  "gene": "UniProtKB:P38567",
  "term_label": "hyaluronan catabolic process"
}